{
  "term_label": "inositol 1,4,5 trisphosphate binding",
  "gene_name": "Short transient receptor potential channel 4",
  "gene_symbol": "TRPC4",
  "gene": "UniProtKB:Q9UBN4",
  "term_id": "GO:0070679"
}